{
  "term_label": "galactose catabolic process",
  "gene_symbol": "GLB1L",
  "term_id": "GO:0019388",
  "gene_name": "Beta-galactosidase-1-like protein",
  "gene": "UniProtKB:Q6UWU2"
}